{
  "gene_name": "ADP-ribosylation factor 6",
  "gene": "UniProtKB:P62330",
  "term_label": "endocytic vesicle",
  "term_id": "GO:0030139",
  "gene_symbol": "ARF6"
}